{
  "gene_symbol": "TMEM258",
  "term_id": "GO:0062062",
  "gene_name": "Transmembrane protein 258",
  "gene": "UniProtKB:P61165",
  "term_label": "oligosaccharyltransferase complex binding"
}